L-glutamate transmembrane export from vacuole [GO:0089704] (biological process) References: PMID:21307582 Relationships: is a type of L-glutamate transmembrane transport [GO:0015813]; is a type of amino acid transmembrane export from vacuole [GO:0032974] Definition: The directed movement of L-glutamate out of the vacuole, across the vacuolar membrane.